{
  "term_id": "GO:0000723",
  "gene_symbol": "HUS1B",
  "gene_name": "Checkpoint protein HUS1B",
  "gene": "UniProtKB:Q8NHY5",
  "term_label": "telomere maintenance"
}